{
  "gene_symbol": "IL17F",
  "gene": "UniProtKB:Q96PD4",
  "term_id": "GO:0097400",
  "gene_name": "Interleukin-17F",
  "term_label": "interleukin-17-mediated signaling pathway"
}